glycine-oxaloacetate transaminase activity [GO:0047303] (molecular function) Definition: Catalysis of the reaction: glycine + oxaloacetate = L-aspartate + glyoxylate. Also known as: glycine-oxaloacetate aminotransferase activity, glycine--oxaloacetate aminotransferase activity, glycine-oxalacetate aminotransferase activity, glycine:oxaloacetate aminotransferase activity Relationships: is_a transaminase activity [GO:0008483] Sources: EC:2.6.1.35, RHEA:17141